{
  "term_id": "UNKNOWN:0002",
  "term_label": "Unknown biological process",
  "gene_symbol": "COL6A3",
  "gene": "UniProtKB:P12111",
  "gene_name": "Collagen alpha-3(VI) chain"
}